membrane addition at site of mitotic cytokinesis [GO:0061796] (biological process) Relationships: is a type of GO:0007107; is a type of GO:1902410 Definition: A mitotic cell cycle process involved in the net addition of membrane at the site of cytokinesis; includes vesicle recruitment and fusion, local lipid synthesis and insertion. Sources: GOC:dph, GOC:vw